{
  "term_id": "GO:0005615",
  "gene": "UniProtKB:P04278",
  "gene_symbol": "SHBG",
  "term_label": "extracellular space",
  "gene_name": "Sex hormone-binding globulin"
}